negative regulation of gastric mucosal blood circulation [GO:1904345] (biological process) Relationships: is a type of negative regulation of blood circulation [GO:1903523]; is a type of GO:1904344; negatively regulates gastric mucosal blood circulation [GO:1990768] Definition: Any process that stops, prevents or reduces the frequency, rate or extent of gastric mucosal blood circulation. References: PMID:10807413 Sources: GOC:TermGenie, GO_REF:0000058 Also known as: down regulation of gastric mucosal blood circulation, down regulation of stomach mucosal blood circulation, down-regulation of gastric mucosal blood circulation, down-regulation of stomach mucosal blood circulation, downregulation of gastric mucosal blood circulation, downregulation of stomach mucosal blood circulation, negative regulation of stomach mucosal blood circulation, inhibition of gastric mucosal blood circulation, inhibition of stomach mucosal blood circulation